glycosome membrane [GO:0046860] (cellular component) Sources: GOC:ai Relationships: is a type of peroxisomal membrane [GO:0005778]; is part of GO:0020015 Definition: The lipid bilayer surrounding a glycosome.